{
  "term_label": "Unknown molecular function",
  "gene_symbol": "TMEM9B",
  "gene": "UniProtKB:Q9NQ34",
  "gene_name": "Transmembrane protein 9B",
  "term_id": "UNKNOWN:0001"
}